{
  "gene_name": "Exostosin-like 1",
  "term_id": "GO:0005794",
  "gene_symbol": "EXTL1",
  "gene": "UniProtKB:Q92935",
  "term_label": "Golgi apparatus"
}